symbiont-mediated activation of host plasminogen [GO:0044542] (biological process) Also known as: plasminogen activation in another organism, plasminogen activation in other organism References: PMID:18070889, PMID:27533300, PMID:34305859 Definition: A process in which a symbiont initiates, promotes, or enhances the normal activation of plasminogen, the pathway resulting in the processing of inactive plasminogen to active plasmin in the host organism. This can facilitate the dissemination of the symbiont into host tissues. It can also be used to destroy complement, opsonins as well as antibacterial proteins like histones. Relationships: is a type of symbiont-mediated perturbation of host cellular process [GO:0044068]